{
  "gene_symbol": "B9D1",
  "term_id": "GO:0036038",
  "gene": "UniProtKB:Q9UPM9",
  "gene_name": "B9 domain-containing protein 1",
  "term_label": "MKS complex"
}